{
  "term_id": "GO:0007218",
  "term_label": "neuropeptide signaling pathway",
  "gene_symbol": "NMB",
  "gene_name": "Neuromedin-B",
  "gene": "UniProtKB:P08949"
}